{
  "term_id": "GO:0008360",
  "term_label": "regulation of cell shape",
  "gene_symbol": "PLXNB3",
  "gene_name": "Plexin-B3",
  "gene": "UniProtKB:Q9ULL4"
}